{
  "term_label": "Unknown molecular function",
  "gene_symbol": "PTCD2",
  "term_id": "UNKNOWN:0001",
  "gene": "UniProtKB:Q8WV60",
  "gene_name": "Pentatricopeptide repeat-containing protein 2, mitochondrial"
}